ureteric bud formation [GO:0060676] (BP) Relationships: is a type of mesonephric tubule formation [GO:0072172]; is part of ureteric bud morphogenesis [GO:0060675] Regulation: regulated by regulation of ureteric bud formation [GO:0072106]; positively regulated by positive regulation of ureteric bud formation [GO:0072107] Definition: The developmental process pertaining to the initial formation of the ureteric bud from the Wolffian duct. This process begins when the bud protrudes from the duct and ends when it is a recognizable bud. References: PMID:16916378 Sources: GOC:dph